{
  "gene_symbol": "UBE2QL1",
  "term_id": "GO:0005634",
  "gene": "UniProtKB:A1L167",
  "term_label": "nucleus",
  "gene_name": "Ubiquitin-conjugating enzyme E2Q-like protein 1"
}